anterior lateral line neuromast hair cell development [GO:0035676] (biological process) Relationships: is a type of neuromast hair cell development [GO:0035675]; is part of anterior lateral line neuromast hair cell differentiation [GO:0048903] Definition: The process whose specific outcome is the progression of an anterior lateral line neuromast hair cell over time, from its formation to the mature structure. A neuromast hair cell is a hair cell that acts as a sensory receptor of the neuromast; it is morphologically polarized as a result of the relative position of the single kinocilium and the clusters of stereocilia on its apical surface. Cell development does not include the steps involved in committing a cell to a specific fate. Sources: ISBN:0125296509, ISBN:0387968377